{
  "term_label": "Unknown molecular function",
  "gene": "UniProtKB:Q5VZQ5",
  "gene_symbol": "TEX36",
  "gene_name": "Testis-expressed protein 36",
  "term_id": "UNKNOWN:0001"
}